{
  "gene_name": "12-(S)-hydroxy-5,8,10,14-eicosatetraenoic acid receptor",
  "gene_symbol": "GPR31",
  "term_label": "G protein-coupled receptor signaling pathway",
  "gene": "UniProtKB:O00270",
  "term_id": "GO:0007186"
}